glucuronylgalactosylproteoglycan 4-beta-N-acetylgalactosaminyltransferase activity [GO:0047237] (molecular function) Also known as: N-acetylgalactosaminyltransferase I activity, glucuronylgalactosylproteoglycan beta-1,4-N-acetylgalactosaminyltransferase activity, UDP-N-acetyl-D-galactosamine:D-glucuronyl-1,3-beta-D-galactosyl-proteoglycan beta-1,4-N-acetylgalactosaminyltransferase activity, uridine diphosphoacetylgalactosamine-chondroitin acetylgalactosaminyltransferase I, uridine diphosphoacetylgalactosamine-chondroitinacetylgalactosaminyltransferase I activity Definition: Catalysis of the reaction: D-glucuronyl-1,3-beta-D-galactosylproteoglycan + UDP-N-acetylgalactosamine = N-acetyl-D-galactosaminyl-1,4-beta-D-glucuronyl-1,3-beta-D-galactosylproteoglycan + UDP. Relationships: is_a acetylgalactosaminyltransferase activity [GO:0008376] Sources: EC:2.4.1.174, MetaCyc:2.4.1.174-RXN